{
  "gene_symbol": "HLA-DPA1",
  "term_label": "peptide antigen assembly with MHC class II protein complex",
  "gene": "UniProtKB:P20036",
  "term_id": "GO:0002503",
  "gene_name": "HLA class II histocompatibility antigen, DP alpha 1 chain"
}